{
  "gene_name": "Probable C-mannosyltransferase DPY19L2",
  "term_label": "nuclear inner membrane",
  "term_id": "GO:0005637",
  "gene_symbol": "DPY19L2",
  "gene": "UniProtKB:Q6NUT2"
}